{
  "gene_symbol": "MIOS",
  "term_label": "positive regulation of TORC1 signaling",
  "gene": "UniProtKB:Q9NXC5",
  "gene_name": "GATOR complex protein MIOS",
  "term_id": "GO:1904263"
}